{
  "term_label": "regulation of transcription by RNA polymerase II",
  "gene_name": "Zinc finger and BTB domain-containing protein 21",
  "gene": "UniProtKB:Q9ULJ3",
  "gene_symbol": "ZBTB21",
  "term_id": "GO:0006357"
}